{
  "gene_name": "Receptor-type tyrosine-protein phosphatase O",
  "gene": "UniProtKB:Q16827",
  "term_label": "regulation of glomerular filtration",
  "gene_symbol": "PTPRO",
  "term_id": "GO:0003093"
}